{
  "term_id": "GO:0000976",
  "term_label": "transcription cis-regulatory region binding",
  "gene_name": "Zinc finger protein 814",
  "gene": "UniProtKB:B7Z6K7",
  "gene_symbol": "ZNF814"
}